transforming growth factor beta production [GO:0071604] (biological process) Relationships: is a type of cytokine production [GO:0001816] Also known as: TGF-B production, TGF-beta production, TGFb production, TGFbeta production, transforming growth factor-beta production, transforming growth factor-beta secretion Definition: The appearance of any member of the transforming growth factor-beta family of cytokines due to biosynthesis or secretion following a cellular stimulus, resulting in an increase in its intracellular or extracellular levels. Transforming growth factor-beta family members include TGF-B1, TGF-B2, and TGF-B3. Regulation: regulated by regulation of transforming growth factor beta production [GO:0071634]; negatively regulated by negative regulation of transforming growth factor beta production [GO:0071635]; RO_0002213 by positive regulation of transforming growth factor beta production [GO:0071636] Subtypes: GO:0032905, GO:0032906, transforming growth factor beta3 production [GO:0032907] References: PMID:16891311, PMID:2022183 Sources: GOC:add, GOC:rv